regulation of intrinsic apoptotic signaling pathway in response to osmotic stress [GO:1902218] (biological process) Subtypes: GO:1902219, GO:1902220, GO:1902238 Definition: Any process that modulates the frequency, rate or extent of intrinsic apoptotic signaling pathway in response to osmotic stress. Relationships: is a type of GO:0106049; is a type of regulation of intrinsic apoptotic signaling pathway [GO:2001242]; RO_0002211 intrinsic apoptotic signaling pathway in response to osmotic stress [GO:0008627] References: PMID:14569084 Sources: GOC:BHF, GOC:TermGenie, GOC:mtg_apoptosis, GOC:rl